{
  "gene": "UniProtKB:P18428",
  "term_label": "lipopolysaccharide-mediated signaling pathway",
  "gene_symbol": "LBP",
  "term_id": "GO:0031663",
  "gene_name": "Lipopolysaccharide-binding protein"
}